{
  "term_id": "UNKNOWN:0003",
  "gene_symbol": "MEF2B",
  "gene_name": "Myocyte-specific enhancer factor 2B",
  "gene": "UniProtKB:Q02080",
  "term_label": "Unknown cellular component"
}